{
  "gene_name": "Olfactory receptor 6N2",
  "term_label": "detection of chemical stimulus involved in sensory perception of smell",
  "gene": "UniProtKB:Q8NGY6",
  "gene_symbol": "OR6N2",
  "term_id": "GO:0050911"
}